oxytocin receptor binding [GO:0031855] (molecular function) Sources: GOC:mah, GOC:nln Definition: Binding to an oxytocin receptor. Relationships: is a type of G protein-coupled receptor binding [GO:0001664] Also known as: oxytocin receptor ligand